{
  "gene": "UniProtKB:Q53QV2",
  "term_label": "Unknown molecular function",
  "gene_name": "Protein LBH",
  "term_id": "UNKNOWN:0001",
  "gene_symbol": "LBH"
}